{
  "gene_name": "Mitotic checkpoint serine_threonine-protein kinase BUB1",
  "term_label": "mitotic spindle assembly checkpoint signaling",
  "gene": "UniProtKB:O43683",
  "gene_symbol": "BUB1",
  "term_id": "GO:0007094"
}